ventricular system development [GO:0021591] (biological process) Definition: The process whose specific outcome is the progression of the brain ventricular system over time, from its formation to the mature structure. The brain ventricular system consists of four communicating cavities within the brain that are continuous with the central canal of the spinal cord. These cavities include two lateral ventricles, the third ventricle and the fourth ventricle. Cerebrospinal fluid fills the ventricles and is produced by the choroid plexus. Relationships: is a type of system development [GO:0048731]; is part of brain development [GO:0007420] Sources: GOC:cls, GOC:dgh, GOC:dph, GOC:jid, GO_REF:0000021